{
  "gene_symbol": "RNH1",
  "term_id": "GO:0045765",
  "gene": "UniProtKB:P13489",
  "term_label": "regulation of angiogenesis",
  "gene_name": "Ribonuclease inhibitor"
}